{
  "term_label": "Unknown molecular function",
  "gene_name": "Calpain small subunit 2",
  "gene_symbol": "CAPNS2",
  "gene": "UniProtKB:Q96L46",
  "term_id": "UNKNOWN:0001"
}